regulation of inflammatory response to antigenic stimulus [GO:0002861] (biological process) Sources: GOC:add Definition: Any process that modulates the frequency, rate, or extent of an inflammatory response to an antigenic stimulus. Subtypes: negative regulation of inflammatory response to antigenic stimulus [GO:0002862], positive regulation of inflammatory response to antigenic stimulus [GO:0002863], regulation of acute inflammatory response to antigenic stimulus [GO:0002864], regulation of chronic inflammatory response to antigenic stimulus [GO:0002874] Relationships: is a type of regulation of inflammatory response [GO:0050727]; is a type of regulation of immune response [GO:0050776]; regulates GO:0002437